aleurone grain lumen [GO:0034422] (CC) Definition: The volume enclosed by the membrane of an aleurone grain. Sources: GOC:rph Relationships: is a type of cytoplasmic vesicle lumen [GO:0060205]; is part of aleurone grain [GO:0033095]